RNA polymerase II sequence-specific DNA-binding transcription factor recruiting activity [GO:0001010] (molecular function) Definition: The function of binding to a specific DNA sequence and recruiting another transcription factor to the DNA in order to modulate transcription. The recruited factor may bind DNA directly, or may be colocalized via protein-protein interactions. Relationships: is_a GO:0030674; has part RNA polymerase II-specific DNA-binding transcription factor binding [GO:0061629] Sources: GOC:txnOH Also known as: sequence-specific DNA binding transcription factor recruiting transcription factor activity, transcription factor activity, sequence-specific DNA binding transcription factor recruiting, transcription factor activity, sequence-specific DNA-binding transcription factor recruiting